phosphatidylcholine biosynthesis from phosphoryl-ethanolamine via N-dimethylethanolamine phosphate and CDP-choline [GO:0070832] (biological process) Definition: The phosphatidylcholine biosynthetic process that begins with three consecutive N-methylation steps that are carried out on phospho-bases, phosphoethanolamine, phospho-N-methylethanolamine, and phospho-N-dimethylethanolamine; the process ends with the conversion of a phosphatidyl-N-dimethylethanolamine to a phosphatidylcholine. Relationships: is a type of phosphatidylcholine biosynthetic process [GO:0006656] Sources: MetaCyc:PWY4FS-2